{
  "term_id": "UNKNOWN:0002",
  "term_label": "Unknown biological process",
  "gene": "UniProtKB:Q8NB46",
  "gene_symbol": "ANKRD52",
  "gene_name": "Serine_threonine-protein phosphatase 6 regulatory ankyrin repeat subunit C"
}